{
  "term_id": "GO:0048793",
  "gene_symbol": "OSR1",
  "gene_name": "Protein odd-skipped-related 1",
  "gene": "UniProtKB:Q8TAX0",
  "term_label": "pronephros development"
}